{
  "term_label": "extracellular space",
  "gene_symbol": "SCGB1D4",
  "gene_name": "Secretoglobin family 1D member 4",
  "term_id": "GO:0005615",
  "gene": "UniProtKB:Q6XE38"
}